defense response to other organism [GO:0098542] (biological process) Also known as: defence response incompatible interaction, defence response to pathogen, incompatible interaction, defense response, incompatible interaction, resistance response to pathogen Definition: Reactions triggered in response to the presence of another organism that act to protect the cell or organism from damage caused by that organism. Relationships: is a type of defense response [GO:0006952]; is_a response to other organism [GO:0051707] Subtypes: GO:0002242, defense response to protozoan [GO:0042832], defense response to symbiont [GO:0140546] Sources: GOC:dos